{
  "gene_name": "Fumarate hydratase, mitochondrial",
  "gene": "UniProtKB:P07954",
  "gene_symbol": "FH",
  "term_id": "GO:0006106",
  "term_label": "fumarate metabolic process"
}